{
  "gene_symbol": "SFSWAP",
  "term_label": "Unknown cellular component",
  "term_id": "UNKNOWN:0003",
  "gene_name": "Splicing factor, suppressor of white-apricot homolog",
  "gene": "UniProtKB:Q12872"
}